{
  "gene_name": "D(1A) dopamine receptor",
  "term_label": "adenylate cyclase-activating adrenergic receptor signaling pathway",
  "gene": "UniProtKB:P21728",
  "term_id": "GO:0071880",
  "gene_symbol": "DRD1"
}